{
  "term_id": "GO:0048013",
  "term_label": "ephrin receptor signaling pathway",
  "gene_name": "Ephrin-B3",
  "gene_symbol": "EFNB3",
  "gene": "UniProtKB:Q15768"
}